T=7 icosahedral viral capsid [GO:0039620] (cellular component) Sources: VZ:804 Relationships: is_a icosahedral viral capsid [GO:0019030] Definition: The protein coat that surrounds the infective nucleic acid in some virus particles where the subunits (capsomeres) are arranged to form an icosahedron with T=7 symmetry. The T=7 capsid is composed of 12 pentameric and 60 hexameric capsomeres. Note: Spherical viruses with T numbers greater than or equal to 7 are skewed. They are therefore described as either right-handed (dextro) or left-handed (laevo).